methylene-fatty-acyl-phospholipid synthase activity [GO:0004481] (molecular function) Sources: EC:2.1.1.16 Relationships: is a type of S-adenosylmethionine-dependent methyltransferase activity [GO:0008757] Definition: Catalysis of the reaction: S-adenosyl-L-methionine + phospholipid olefinic fatty acid = S-adenosyl-L-homocysteine + phospholipid methylene fatty acid. Also known as: cyclopropane synthetase activity, unsaturated-phospholipid methyltransferase activity, S-adenosyl-L-methionine:unsaturated-phospholipid methyltransferase (methenylating)